omega-hydroxyceramide biosynthetic process [GO:0106342] (biological process) Definition: The chemical reactions and pathways resulting in the formation of omega-hydroxyceramide/acylceramide. Relationships: is a type of ceramide biosynthetic process [GO:0046513] References: PMID:28248318